{
  "term_label": "triglyceride catabolic process",
  "gene_name": "Patatin-like phospholipase domain-containing protein 5",
  "gene": "UniProtKB:Q7Z6Z6",
  "term_id": "GO:0019433",
  "gene_symbol": "PNPLA5"
}